{
  "gene": "UniProtKB:Q8NFQ5",
  "term_label": "Unknown cellular component",
  "term_id": "UNKNOWN:0003",
  "gene_name": "BPI fold-containing family B member 6",
  "gene_symbol": "BPIFB6"
}